{
  "term_label": "Unknown molecular function",
  "term_id": "UNKNOWN:0001",
  "gene_name": "Mitochondrial import inner membrane translocase subunit Tim8 B",
  "gene": "UniProtKB:Q9Y5J9",
  "gene_symbol": "TIMM8B"
}